alphaV-beta8 integrin-MMP14-TGFbeta-1 complex [GO:0071100] (cellular component) Relationships: is a type of plasma membrane protein complex [GO:0098797] Definition: A protein complex that consists of an alphaV-beta8 integrin complex bound to matrix metalloproteinase 14 and transforming growth factor beta-1 (TGFbeta-1). Also known as: ITGAV-ITGB8-MMP14-TGFB1 complex References: PMID:11970960